bronchiole morphogenesis [GO:0060436] (biological process) Relationships: is a type of tube morphogenesis [GO:0035239]; is part of bronchiole development [GO:0060435] Definition: The process in which a bronchiole is generated and organized. A bronchiole is the first airway branch that no longer contains cartilage; it is a branch of the bronchi. Sources: GOC:dph